post-embryonic development [GO:0009791] (biological process) Subtypes: larval development [GO:0002164], instar larval or pupal development [GO:0002165], photomorphogenesis [GO:0009640], GO:0009647, acquisition of plant reproductive competence [GO:0010049], vegetative phase change [GO:0010050], GO:0010311, GO:0010374, seed development [GO:0048316], fruit septum development [GO:0080127], seedling development [GO:0090351], reproductive shoot system development [GO:0090567], post-embryonic plant organ development [GO:0090696], thermomorphogenesis [GO:0140919], fruit replum development [GO:1990058], GO:1990059 Definition: The process whose specific outcome is the progression of the organism over time, from the completion of embryonic development to the mature structure. See embryonic development. Regulation: regulated by regulation of post-embryonic development [GO:0048580]; negatively regulated by GO:0048581; positively regulated by GO:0048582 Relationships: is a type of multicellular organismal process [GO:0032501]; is part of multicellular organism development [GO:0007275] Sources: GOC:go_curators